{
  "gene_symbol": "CLEC17A",
  "term_id": "GO:0006955",
  "term_label": "immune response",
  "gene_name": "C-type lectin domain family 17, member A",
  "gene": "UniProtKB:Q6ZS10"
}